{
  "term_id": "GO:0006959",
  "term_label": "humoral immune response",
  "gene_name": "Interferon omega-1",
  "gene_symbol": "IFNW1",
  "gene": "UniProtKB:P05000"
}